{
  "gene_name": "Calcium_calmodulin-dependent protein kinase kinase 2",
  "gene_symbol": "CAMKK2",
  "term_label": "CAMKK-AMPK signaling cascade",
  "gene": "UniProtKB:Q96RR4",
  "term_id": "GO:0061762"
}